{
  "term_label": "Unknown cellular component",
  "gene_symbol": "PUS10",
  "term_id": "UNKNOWN:0003",
  "gene_name": "tRNA pseudouridine synthase Pus10",
  "gene": "UniProtKB:Q3MIT2"
}